follicular dendritic cell activation [GO:0002266] (biological process) Definition: A change in the morphology or behavior of a follicular dendritic cell resulting from exposure to an activating factor such as a cellular or soluble ligand. References: PMID:15606789 Sources: GOC:add Subtypes: follicular dendritic cell activation involved in immune response [GO:0002267], follicular dendritic cell differentiation [GO:0002268] Relationships: is a type of cell activation [GO:0001775]